{
  "gene_name": "Double-stranded RNA-binding protein Staufen homolog 1",
  "term_label": "mRNA binding",
  "term_id": "GO:0003729",
  "gene": "UniProtKB:O95793",
  "gene_symbol": "STAU1"
}